{
  "gene": "UniProtKB:Q8TE56",
  "gene_name": "A disintegrin and metalloproteinase with thrombospondin motifs 17",
  "term_id": "GO:0031012",
  "term_label": "extracellular matrix",
  "gene_symbol": "ADAMTS17"
}